{
  "term_id": "GO:0005886",
  "gene_symbol": "OR6C2",
  "gene_name": "Olfactory receptor 6C2",
  "term_label": "plasma membrane",
  "gene": "UniProtKB:Q9NZP2"
}